{
  "gene_symbol": "NDUFS7",
  "term_id": "GO:0008137",
  "gene_name": "NADH dehydrogenase [ubiquinone] iron-sulfur protein 7, mitochondrial",
  "term_label": "NADH dehydrogenase (ubiquinone) activity",
  "gene": "UniProtKB:O75251"
}